pro-T cell lineage commitment [GO:0002680] (biological process) Also known as: pro-T cell fate commitment, pro-T lymphocyte fate commitment, pro-T lymphocyte lineage commitment Sources: GOC:add, ISBN:0781735149 Definition: The process in which a lymphoid progenitor cell becomes committed to becoming a pro-T cell. Relationships: is_a GO:0045165; is part of pro-T cell differentiation [GO:0002572]